alpha-1,2-galactosyltransferase activity [GO:0031278] (molecular function) Definition: Catalysis of the transfer of a galactose residue from a donor molecule, such as GDP-galactose or UDP-galactose, to an oligosaccharide, forming an alpha-1,2-linkage. References: PMID:7522655 Relationships: is a type of galactosyltransferase activity [GO:0008378]